oxysterol transfer activity [GO:0120021] (molecular function) References: PMID:20823909, PMID:24220498, PMID:25797198 Sources: GOC:krc Also known as: oxysterol carrier activity, intermembrane oxysterol transfer activity Relationships: is a type of sterol transfer activity [GO:0120015]; has part GO:0008142 Definition: Removes oxysterol from a membrane or a monolayer lipid particle, transports it through the aqueous phase while protected in a hydrophobic pocket, and brings it to an acceptor membrane or lipid particle.